pre-replicative complex assembly involved in nuclear cell cycle DNA replication [GO:0006267] (biological process) Sources: GOC:mtg_cell_cycle Relationships: is a type of pre-replicative complex assembly involved in cell cycle DNA replication [GO:1902299]; is part of GO:0033260 Definition: The aggregation, arrangement and bonding together of a set of components to form the nuclear pre-replicative complex, a protein-DNA complex that forms at the eukaryotic DNA replication origin and is required for replication initiation. Subtypes: GO:1902984, mitotic pre-replicative complex assembly [GO:1902985] Also known as: pre-RC complex assembly, pre-replicative complex assembly, pre-replicative complex formation, nuclear pre-replicative complex assembly